{
  "term_label": "nuclear envelope",
  "gene_name": "Importin-7",
  "term_id": "GO:0005635",
  "gene": "UniProtKB:O95373",
  "gene_symbol": "IPO7"
}